{
  "gene_symbol": "TBC1D3B",
  "term_label": "Unknown biological process",
  "gene_name": "TBC1 domain family member 3B",
  "term_id": "UNKNOWN:0002",
  "gene": "UniProtKB:A6NDS4"
}